{
  "gene": "UniProtKB:P51888",
  "term_id": "UNKNOWN:0002",
  "term_label": "Unknown biological process",
  "gene_symbol": "PRELP",
  "gene_name": "Prolargin"
}